{
  "term_id": "GO:0000795",
  "gene_symbol": "SYCE1L",
  "term_label": "synaptonemal complex",
  "gene_name": "Synaptonemal complex central element protein 1-like",
  "gene": "UniProtKB:A8MT33"
}